{
  "gene_name": "Cytochrome P450 1A2",
  "gene": "UniProtKB:P05177",
  "term_id": "GO:0016712",
  "gene_symbol": "CYP1A2",
  "term_label": "oxidoreductase activity, acting on paired donors, with incorporation or reduction of molecular oxygen, reduced flavin or flavoprotein as one donor, and incorporation of one atom of oxygen"
}